{
  "term_label": "RNA polymerase II cis-regulatory region sequence-specific DNA binding",
  "gene_symbol": "RFX6",
  "gene_name": "DNA-binding protein RFX6",
  "term_id": "GO:0000978",
  "gene": "UniProtKB:Q8HWS3"
}